negative regulation of urothelial cell proliferation [GO:0050676] (biological process) Definition: Any process that stops, prevents or reduces the rate or extent of urothelial cell proliferation. Also known as: down regulation of urothelial cell proliferation, down-regulation of urothelial cell proliferation, downregulation of urothelial cell proliferation, inhibition of urothelial cell proliferation Sources: GOC:ai Relationships: is a type of GO:0050675; is_a negative regulation of epithelial cell proliferation [GO:0050680]; negatively regulates GO:0050674